{
  "term_id": "GO:0005615",
  "gene_name": "Macrophage colony-stimulating factor 1",
  "gene": "UniProtKB:P09603",
  "term_label": "extracellular space",
  "gene_symbol": "CSF1"
}